{
  "term_id": "GO:0003779",
  "gene": "UniProtKB:Q12929",
  "gene_name": "Epidermal growth factor receptor kinase substrate 8",
  "gene_symbol": "EPS8",
  "term_label": "actin binding"
}